{
  "gene": "UniProtKB:Q9NRD5",
  "gene_symbol": "PICK1",
  "gene_name": "PRKCA-binding protein",
  "term_id": "GO:0043113",
  "term_label": "receptor clustering"
}